{
  "gene": "UniProtKB:P30531",
  "gene_name": "Sodium- and chloride-dependent GABA transporter 1",
  "term_id": "GO:0030424",
  "gene_symbol": "SLC6A1",
  "term_label": "axon"
}